{
  "term_label": "endosomal transport",
  "term_id": "GO:0016197",
  "gene": "UniProtKB:O94876",
  "gene_symbol": "TMCC1",
  "gene_name": "Transmembrane and coiled-coil domains protein 1"
}